histamine secretion mediated by IgE immunoglobulin [GO:0097279] (biological process) Sources: GOC:add, GOC:rv Relationships: is a type of histamine secretion mediated by immunoglobulin [GO:0097280] Also known as: Ig-mediated histamine release, histamine secretion mediated by IgE antibody Definition: Histamine release triggered by the binding of an antigen to an IgE immunoglobulin bound to the cell surface. An example is mast cell histamine degranulation as a result of exposure of mast cell-bound IgE to alder tree pollen.